triacylglycerol lipase activity [GO:0004806] (molecular function) Definition: Catalysis of the reaction: a triacylglycerol + H2O = a diacylglycerol + a fatty acid + H+. Sources: RHEA:12044 Also known as: TAG activity, triglyceride lipase activity, heparin releasable hepatic lipase, hepatic lipase, hepatic monoacylglycerol acyltransferase, liver lipase, post-heparin plasma protamine-resistant lipase, salt-resistant post-heparin lipase, GA 56, GEH, PPL, amano AP, amano B, amano CE, amano CES, amano P, amno N-AP, butyrinase activity, cacordase activity, capalase L, glycerol ester hydrolase activity, glycerol-ester hydrolase activity, lipazin, meito MY 30, meito sangyo OF lipase, steapsin, takedo 1969-4-9, triacetinase activity, triacylglycerol acylhydrolase activity, triacylglycerol ester hydrolase activity, tributyrase activity, tributyrin esterase activity, tributyrinase activity, triglyceridase activity, triglyceride hydrolase activity, triolein hydrolase activity, tween hydrolase activity, tween-hydrolyzing esterase activity, tweenase activity, tweenesterase activity Relationships: is_a lipase activity [GO:0016298]; is a type of GO:0052689 Subtypes: lipoprotein lipase activity [GO:0004465] Regulation: positively regulated by GO:0061365